protopanaxadiol 6-hydroxylase activity [GO:0102557] (molecular function) Definition: Catalysis of the reaction: (20S)-protopanaxadiol + O2 + reduced [NADPH--hemoprotein reductase] = (20S)-protopanaxatriol + H+ + H2O + oxidized [NADPH--hemoprotein reductase]. Sources: EC:1.14.14.121 Relationships: is a type of oxidoreductase activity, acting on paired donors, with incorporation or reduction of molecular oxygen, NAD(P)H as one donor, and incorporation of one atom of oxygen [GO:0016709]